{
  "gene_name": "Histone-arginine methyltransferase METTL23",
  "gene": "UniProtKB:Q86XA0",
  "term_id": "GO:0040029",
  "term_label": "epigenetic regulation of gene expression",
  "gene_symbol": "METTL23"
}